intronic box C/D snoRNA processing [GO:0034965] (biological process) Sources: GOC:krc, GOC:mah Definition: Any process involved in the conversion of a primary box C/D type small nucleolar RNA (snoRNA) transcript that resides within, and is processed from, the intron of a pre-mRNA into a mature box C/D snoRNA. Relationships: is a type of GO:0031070; is_a box C/D sno(s)RNA processing [GO:0034963]